restriction endodeoxyribonuclease activity [GO:0015666] (MF) Definition: Catalysis of endonucleolytic cleavage of DNA in a site-specific manner, resulting in double-strand breaks. Sources: GOC:mlg Subtypes: GO:0009035, type II site-specific deoxyribonuclease activity [GO:0009036], type III site-specific deoxyribonuclease activity [GO:0015668], GO:0032067 Relationships: is a type of DNA endonuclease activity [GO:0004520]; is a type of hydrolase activity, acting on ester bonds [GO:0016788] Also known as: restriction endonuclease activity, restriction enzyme activity